{
  "gene_name": "Transient receptor potential cation channel subfamily M member 6",
  "term_label": "protein kinase activity",
  "gene": "UniProtKB:Q9BX84",
  "term_id": "GO:0004672",
  "gene_symbol": "TRPM6"
}